{
  "gene": "UniProtKB:Q99633",
  "term_id": "GO:0000350",
  "gene_symbol": "PRPF18",
  "gene_name": "Pre-mRNA-splicing factor 18",
  "term_label": "generation of catalytic spliceosome for second transesterification step"
}